protein-N(pi)-phosphohistidine--N-acetyl-D-glucosamine phosphotransferase activity [GO:0103111] (molecular function) Also known as: D-glucosamine PTS permease activity, N-acetyl-D-glucosamine PTS permease activity Sources: RHEA:49240 Relationships: is a type of GO:0016773 Definition: Catalysis of the reaction: N(pros)-phospho-L-histidyl-[protein] + N-acetyl-D-glucosamine(out) = L-histidyl-[protein] + N-acetyl-D-glucosamine 6-phosphate(in).